{
  "term_id": "UNKNOWN:0002",
  "gene_symbol": "GTPBP8",
  "term_label": "Unknown biological process",
  "gene_name": "GTP-binding protein 8",
  "gene": "UniProtKB:Q8N3Z3"
}